{
  "gene_symbol": "SPNS2",
  "gene_name": "Sphingosine-1-phosphate transporter SPNS2",
  "gene": "UniProtKB:Q8IVW8",
  "term_id": "GO:0016020",
  "term_label": "membrane"
}